{
  "gene_name": "Testis-specific chromodomain protein Y 1",
  "gene": "UniProtKB:Q9Y6F8",
  "term_id": "GO:0061628",
  "gene_symbol": "CDY1B",
  "term_label": "histone H3K27me3 reader activity"
}